negative regulation of muscle hyperplasia [GO:0014740] (biological process) Relationships: is a type of regulation of muscle hyperplasia [GO:0014738]; is a type of GO:0014745; negatively regulates muscle hyperplasia [GO:0014900] Definition: Any process that stops, prevents, or reduces the frequency, rate, or extent of muscle hyperplasia. Sources: GOC:mtg_muscle